{
  "gene_symbol": "PLET1",
  "term_id": "GO:0001953",
  "gene": "UniProtKB:Q6UQ28",
  "gene_name": "Placenta-expressed transcript 1 protein",
  "term_label": "negative regulation of cell-matrix adhesion"
}